negative regulation of conjugation with zygote [GO:0140538] (biological process) Definition: A process that prevents a zygote from fusing an additional cell. Relationships: is a type of GO:0031138 References: PMID:30089908